response to external biotic stimulus [GO:0043207] (biological process) Sources: GOC:go_curators Relationships: is a type of response to external stimulus [GO:0009605]; is a type of response to biotic stimulus [GO:0009607] Subtypes: response to molecule of bacterial origin [GO:0002237], response to molecule of fungal origin [GO:0002238], GO:0002240, response to other organism [GO:0051707], cellular response to external biotic stimulus [GO:0071217], GO:0098581 Definition: Any process that results in a change in state or activity of a cell or an organism (in terms of movement, secretion, enzyme production, gene expression, etc.) as a result of an external biotic stimulus, an external stimulus caused by, or produced by living things.